{
  "term_label": "synaptic vesicle clustering",
  "gene": "UniProtKB:Q92777",
  "gene_symbol": "SYN2",
  "gene_name": "Synapsin-2",
  "term_id": "GO:0097091"
}